inner ear morphogenesis [GO:0042472] (biological process) Definition: The process in which the anatomical structures of the inner ear are generated and organized. The inner ear is the structure in vertebrates that contains the organs of balance and hearing. It consists of soft hollow sensory structures (the membranous labyrinth) containing fluid (endolymph) surrounded by fluid (perilymph) and encased in a bony cavity (the bony labyrinth). It consists of two chambers, the sacculus and utriculus, from which arise the cochlea and semicircular canals respectively. Subtypes: otic vesicle morphogenesis [GO:0071600] Sources: GOC:jl, ISBN:0192801023 Relationships: is a type of embryonic morphogenesis [GO:0048598]; is part of GO:0042471; is part of inner ear development [GO:0048839]